{
  "gene": "UniProtKB:P15813",
  "gene_symbol": "CD1D",
  "term_label": "exogenous lipid antigen binding",
  "term_id": "GO:0030884",
  "gene_name": "Antigen-presenting glycoprotein CD1d"
}